{
  "gene_name": "Membrane-spanning 4-domains subfamily A member 13",
  "term_id": "UNKNOWN:0001",
  "gene_symbol": "MS4A13",
  "term_label": "Unknown molecular function",
  "gene": "UniProtKB:Q5J8X5"
}